{
  "gene_name": "Protein mono-ADP-ribosyltransferase PARP3",
  "term_id": "GO:0005730",
  "term_label": "nucleolus",
  "gene": "UniProtKB:Q9Y6F1",
  "gene_symbol": "PARP3"
}